{
  "gene": "UniProtKB:Q15046",
  "term_id": "GO:0004824",
  "gene_name": "Lysine--tRNA ligase",
  "term_label": "lysine-tRNA ligase activity",
  "gene_symbol": "KARS1"
}